{
  "gene": "UniProtKB:Q5MIZ7",
  "gene_symbol": "PPP4R3B",
  "term_id": "GO:0005654",
  "term_label": "nucleoplasm",
  "gene_name": "Serine_threonine-protein phosphatase 4 regulatory subunit 3B"
}